glycol catabolic process [GO:0042846] (biological process) Subtypes: GO:0034078, GO:0051144 Relationships: is a type of diol catabolic process [GO:0034313]; is a type of GO:0042844 Definition: The chemical reactions and pathways resulting in the breakdown of glycol, a diol in which the two hydroxy groups are on different carbon atoms, usually but not necessarily adjacent. Sources: Wikipedia:Ethylene_glycol Also known as: dihydric alcohol catabolic process, dihydric alcohol catabolism, glycol breakdown, glycol catabolism, glycol degradation